{
  "gene_name": "5-hydroxytryptamine receptor 3B",
  "gene": "UniProtKB:O95264",
  "term_label": "excitatory extracellular ligand-gated monoatomic ion channel activity",
  "gene_symbol": "HTR3B",
  "term_id": "GO:0005231"
}